negative regulation of cell migration involved in sprouting angiogenesis [GO:0090051] (biological process) Relationships: is a type of negative regulation of blood vessel endothelial cell migration [GO:0043537]; is a type of GO:0090049; negatively regulates cell migration involved in sprouting angiogenesis [GO:0002042] Sources: GOC:BHF, GOC:dph, GOC:rl, GOC:tb Definition: Any process that decreases the frequency, rate or extent of cell migration involved in sprouting angiogenesis. Cell migration involved in sprouting angiogenesis is the orderly movement of endothelial cells into the extracellular matrix in order to form new blood vessels contributing to the process of sprouting angiogenesis.